{
  "gene_name": "Elongation of very long chain fatty acids protein 2",
  "term_id": "GO:0019367",
  "term_label": "fatty acid elongation, saturated fatty acid",
  "gene": "UniProtKB:Q9NXB9",
  "gene_symbol": "ELOVL2"
}